{
  "term_id": "GO:0005737",
  "gene": "UniProtKB:Q00536",
  "gene_name": "Cyclin-dependent kinase 16",
  "term_label": "cytoplasm",
  "gene_symbol": "CDK16"
}